{
  "term_label": "secretory granule membrane",
  "gene_name": "Inositol 1,4,5-trisphosphate receptor type 1",
  "gene": "UniProtKB:Q14643",
  "term_id": "GO:0030667",
  "gene_symbol": "ITPR1"
}